{
  "gene_symbol": "LRFN4",
  "gene": "UniProtKB:Q6PJG9",
  "term_label": "synaptic membrane adhesion",
  "gene_name": "Leucine-rich repeat and fibronectin type-III domain-containing protein 4",
  "term_id": "GO:0099560"
}